pharynx development [GO:0060465] (biological process) Definition: The biological process whose specific outcome is the progression of a pharynx from an initial condition to its mature state. The pharynx is the part of the digestive system immediately posterior to the mouth. Also known as: pharyngeal development Relationships: is_a GO:0048856; is part of GO:0048565 Sources: GOC:dph, GOC:rk Subtypes: chordate pharynx development [GO:0160093], GO:0160094, insect pharynx development [GO:0160095]